DNA synthesis involved in DNA repair [GO:0000731] (biological process) Also known as: DNA repair synthesis, mitotic DNA repair synthesis, DNA synthesis during DNA repair References: PMID:10357855 Relationships: is a type of GO:0071897; is part of GO:0006281 Definition: Synthesis of DNA that proceeds from the broken 3' single-strand DNA end and uses the homologous intact duplex as the template. Subtypes: GO:0000711, DNA synthesis involved in double-strand break repair via homologous recombination [GO:0043150], DNA synthesis involved in double-strand break repair via single-strand annealing [GO:0043151], DNA synthesis involved in UV-damage excision repair [GO:1904161]